{
  "gene_name": "Plexin-A4",
  "gene": "UniProtKB:Q9HCM2",
  "gene_symbol": "PLXNA4",
  "term_id": "GO:0071526",
  "term_label": "semaphorin-plexin signaling pathway"
}